{
  "gene_symbol": "LMAN2L",
  "gene_name": "VIP36-like protein",
  "gene": "UniProtKB:Q9H0V9",
  "term_label": "endoplasmic reticulum-Golgi intermediate compartment",
  "term_id": "GO:0005793"
}